{
  "term_id": "GO:0019814",
  "gene_name": "Immunoglobulin kappa variable 2-29",
  "term_label": "immunoglobulin complex",
  "gene": "UniProtKB:A2NJV5",
  "gene_symbol": "IGKV2-29"
}